{
  "term_id": "GO:0006412",
  "gene_symbol": "RPS4X",
  "gene": "UniProtKB:P62701",
  "gene_name": "Small ribosomal subunit protein eS4, X isoform",
  "term_label": "translation"
}